cis-1,2-dihydroxy-4-methylcyclohexa-3,5-diene-1-carboxylate dehydrogenase activity [GO:0018520] (molecular function) Also known as: 4-methylcyclohexa-3,5-diene-1,2-cis-diol-1-carboxylic acid dehydrogenase activity, cis-1,2-dihydroxy-4-methylcyclohexa-3,5-diene-1-carboxylate:NAD(P)+ oxidoreductase (decarboxylating) Definition: Catalysis of the reaction: cis-1,2-dihydroxy-4-methylcyclohexa-3,5-diene-1-carboxylate + NADP+ = 4-methylcatechol + NADPH + H+ + CO2. Relationships: is a type of oxidoreductase activity, acting on the CH-CH group of donors, NAD or NADP as acceptor [GO:0016628] Sources: EC:1.3.1.67